{
  "term_label": "positive regulation of skeletal muscle fiber development",
  "term_id": "GO:0048743",
  "gene_symbol": "MYOG",
  "gene": "UniProtKB:P15173",
  "gene_name": "Myogenin"
}